{
  "term_label": "focal adhesion",
  "gene_symbol": "ITGBL1",
  "gene": "UniProtKB:O95965",
  "term_id": "GO:0005925",
  "gene_name": "Integrin beta-like protein 1"
}